{
  "gene_name": "DDB1- and CUL4-associated factor 1",
  "term_label": "nuclear estrogen receptor binding",
  "gene_symbol": "DCAF1",
  "term_id": "GO:0030331",
  "gene": "UniProtKB:Q9Y4B6"
}